{
  "gene": "UniProtKB:P28223",
  "term_id": "GO:0004993",
  "gene_name": "5-hydroxytryptamine receptor 2A",
  "term_label": "G protein-coupled serotonin receptor activity",
  "gene_symbol": "HTR2A"
}